{
  "gene_symbol": "PRO1716",
  "term_label": "Unknown cellular component",
  "gene": "UniProtKB:Q9UHU1",
  "gene_name": "Putative uncharacterized protein PRO1716",
  "term_id": "UNKNOWN:0003"
}